efferent axon development in posterior lateral line nerve [GO:0048929] (biological process) Definition: The process whose specific outcome is the progression of an efferent axon in the posterior lateral line nerve over time from its formation to the mature structure. This process includes axonogenesis and pathfinding of the efferent axons in the posterior lateral line nerve. References: PMID:15018940 Relationships: is a type of GO:0048894; BFO_0000050 GO:0048918